invagination involved in gastrulation with mouth forming second [GO:0055109] (biological process) Relationships: is a type of embryonic morphogenesis [GO:0048598]; is a type of GO:0060571; is part of gastrulation with mouth forming second [GO:0001702] Definition: The infolding of the epithelial sheet into the embryo involved in deuterostomic gastrulation. Sources: ISBN:0878932437